{
  "gene": "UniProtKB:Q8TBX8",
  "gene_name": "Phosphatidylinositol 5-phosphate 4-kinase type-2 gamma",
  "term_label": "plasma membrane",
  "term_id": "GO:0005886",
  "gene_symbol": "PIP4K2C"
}